{
  "gene_symbol": "DPF1",
  "gene_name": "Zinc finger protein neuro-d4",
  "gene": "UniProtKB:Q92782",
  "term_id": "GO:1990837",
  "term_label": "sequence-specific double-stranded DNA binding"
}